regulation of double-strand break repair via break-induced replication [GO:1901591] (biological process) Definition: Any process that modulates the frequency, rate or extent of double-strand break repair via break-induced replication. Sources: GOC:TermGenie Relationships: is a type of regulation of double-strand break repair via homologous recombination [GO:0010569]; RO_0002211 GO:0000727 Subtypes: negative regulation of double-strand break repair via break-induced replication [GO:1901592]